{
  "term_label": "negative regulation of transcription by RNA polymerase II",
  "gene_symbol": "NR2E1",
  "gene_name": "Nuclear receptor subfamily 2 group E member 1",
  "gene": "UniProtKB:Q9Y466",
  "term_id": "GO:0000122"
}